ICAM-3 receptor activity [GO:0030369] (molecular function) References: PMID:7515813 Sources: GOC:ai, GOC:signaling, ISBN:0198506732 Definition: Combining with ICAM-3, intercellular adhesion molecule 3, and transmitting the signal from one side of the membrane to the other to initiate a change in cell activity. ICAM-3, or CD50, are constitutively expressed on monocytes, granulocytes and lymphocytes; on physiological stimulation, they become transiently phosphorylated on serine residues. Note: Note that this term represents an activity and not a gene product. Consider also annotating to the molecular function terms 'cell adhesion molecule binding ; GO:0050839' and 'receptor binding ; GO:0005102' and the biological process term 'cell adhesion ; GO:0007155'. Relationships: is a type of transmembrane signaling receptor activity [GO:0004888]